catalytic step 2 spliceosome [GO:0071013] (cellular component) References: PMID:18322460, PMID:19239890 Sources: GOC:ab, GOC:krc, GOC:mah, ISBN:0879695897, ISBN:0879697393 Relationships: is a type of GO:0005681; is a type of GO:1902494; BFO_0000051 GO:0000974; has part U5 snRNP [GO:0005682] Subtypes: GO:0071007, U12-type catalytic step 2 spliceosome [GO:0071018] Definition: A spliceosomal complex that contains three snRNPs, including U5, bound to a splicing intermediate in which the first catalytic cleavage of the 5' splice site has occurred. The precise subunit composition differs significantly from that of the catalytic step 1, or activated, spliceosome, and includes many proteins in addition to those found in the associated snRNPs. Also known as: mammalian spliceosomal complex C, mammalian spliceosomal complex C1, yeast spliceosomal complex A2-2